{
  "gene_symbol": "ZNF550",
  "gene_name": "Zinc finger protein 550",
  "term_id": "GO:0005634",
  "term_label": "nucleus",
  "gene": "UniProtKB:Q7Z398"
}